{
  "term_id": "GO:0019448",
  "gene_symbol": "CDO1",
  "term_label": "L-cysteine catabolic process",
  "gene": "UniProtKB:Q16878",
  "gene_name": "Cysteine dioxygenase type 1"
}